{
  "gene_name": "ADP-ribosylation factor-like protein 4C",
  "gene": "UniProtKB:P56559",
  "term_label": "cytoplasm",
  "term_id": "GO:0005737",
  "gene_symbol": "ARL4C"
}